{
  "gene_symbol": "KCNG2",
  "term_label": "membrane",
  "gene_name": "Potassium voltage-gated channel subfamily G member 2",
  "gene": "UniProtKB:Q9UJ96",
  "term_id": "GO:0016020"
}